{
  "gene": "UniProtKB:O15205",
  "term_label": "positive regulation of apoptotic process",
  "gene_name": "Ubiquitin D",
  "gene_symbol": "UBD",
  "term_id": "GO:0043065"
}